{
  "gene_name": "Nuclear autoantigenic sperm protein",
  "term_id": "GO:0042393",
  "gene": "UniProtKB:P49321",
  "gene_symbol": "NASP",
  "term_label": "histone binding"
}